{
  "term_label": "nucleus",
  "gene_name": "Early growth response protein 1",
  "term_id": "GO:0005634",
  "gene_symbol": "EGR1",
  "gene": "UniProtKB:P18146"
}